{
  "gene_name": "Macrophage-capping protein",
  "gene": "UniProtKB:P40121",
  "gene_symbol": "CAPG",
  "term_label": "actin cytoskeleton",
  "term_id": "GO:0015629"
}